{
  "gene_symbol": "NUDT7",
  "gene": "UniProtKB:P0C024",
  "term_id": "GO:0015938",
  "gene_name": "Peroxisomal coenzyme A diphosphatase NUDT7",
  "term_label": "coenzyme A catabolic process"
}